{
  "term_label": "regulation of androgen receptor signaling pathway",
  "gene": "UniProtKB:Q14151",
  "gene_symbol": "SAFB2",
  "term_id": "GO:0060765",
  "gene_name": "Scaffold attachment factor B2"
}